{
  "gene": "UniProtKB:Q9H8U3",
  "term_label": "Unknown cellular component",
  "gene_symbol": "ZFAND3",
  "term_id": "UNKNOWN:0003",
  "gene_name": "AN1-type zinc finger protein 3"
}